{
  "gene_name": "Anterior gradient protein 3",
  "term_label": "dystroglycan binding",
  "term_id": "GO:0002162",
  "gene_symbol": "AGR3",
  "gene": "UniProtKB:Q8TD06"
}